{
  "gene_symbol": "NFYA",
  "term_id": "GO:0006357",
  "term_label": "regulation of transcription by RNA polymerase II",
  "gene": "UniProtKB:P23511",
  "gene_name": "Nuclear transcription factor Y subunit alpha"
}